{
  "term_label": "neuropeptide signaling pathway",
  "gene": "UniProtKB:O00253",
  "term_id": "GO:0007218",
  "gene_name": "Agouti-related protein",
  "gene_symbol": "AGRP"
}